{
  "term_label": "Unknown cellular component",
  "gene": "UniProtKB:A6NGG3",
  "term_id": "UNKNOWN:0003",
  "gene_name": "Putative uncharacterized protein encoded by LINC03041",
  "gene_symbol": "LINC03041"
}